{
  "gene_symbol": "FAAH",
  "term_label": "fatty acid amide hydrolase activity",
  "term_id": "GO:0017064",
  "gene": "UniProtKB:O00519",
  "gene_name": "Fatty-acid amide hydrolase 1"
}